{
  "term_label": "Unknown cellular component",
  "gene_name": "Solute carrier family 22 member 13",
  "term_id": "UNKNOWN:0003",
  "gene_symbol": "SLC22A13",
  "gene": "UniProtKB:Q9Y226"
}